beta-catenin-TCF complex [GO:1990907] (cellular component) References: PMID:11751639, PMID:16936075, PMID:20123964, PMID:21075118, PMID:9419974 Sources: GOC:PARL, GOC:bf Subtypes: beta-catenin-TCF7L2 complex [GO:0070369] Relationships: is a type of RNA polymerase II transcription regulator complex [GO:0090575] Definition: A protein complex that contains beta-catenin and a member of the T-cell factor (TCF)/lymphoid enhancer binding factor (LEF) family of transcription factors. Also known as: beta-catenin/LEF complex, beta-catenin/T-cell factor complex, beta-catenin/lymphoid enhancer binding factor complex